astrocyte fate commitment [GO:0060018] (biological process) Subtypes: forebrain astrocyte fate commitment [GO:0021878] Definition: The commitment of a cells to a specific astrocyte fate and its restriction to develop only into an astrocyte. Sources: GOC:dph Relationships: is a type of glial cell fate commitment [GO:0021781]; is part of astrocyte differentiation [GO:0048708]